{
  "term_label": "endoplasmic reticulum membrane",
  "term_id": "GO:0005789",
  "gene": "UniProtKB:Q5VWC8",
  "gene_symbol": "HACD4",
  "gene_name": "Very-long-chain (3R)-3-hydroxyacyl-CoA dehydratase 4"
}